{
  "gene": "UniProtKB:Q8IV32",
  "term_id": "UNKNOWN:0001",
  "gene_symbol": "CCDC71",
  "term_label": "Unknown molecular function",
  "gene_name": "Coiled-coil domain-containing protein 71"
}